endoplasmic reticulum-endosome membrane contact site [GO:0140284] (cellular component) References: PMID:24105263, PMID:30220460 Definition: A contact site between the endoplasmic reticulum membrane and the endosome membrane. Also known as: ER-endosome membrane contact site Relationships: is a type of organelle membrane contact site [GO:0044232]